regulation of T cell activation via T cell receptor contact with antigen bound to MHC molecule on antigen presenting cell [GO:2001188] (biological process) Subtypes: negative regulation of T cell activation via T cell receptor contact with antigen bound to MHC molecule on antigen presenting cell [GO:2001189], GO:2001190 Relationships: is a type of GO:0002697; is a type of regulation of immune response [GO:0050776]; is a type of regulation of T cell activation [GO:0050863]; RO_0002211 T cell activation via T cell receptor contact with antigen bound to MHC molecule on antigen presenting cell [GO:0002291] Sources: GOC:obol Also known as: regulation of T lymphocyte activation via T cell receptor contact with antigen bound to MHC molecule on antigen presenting cell, regulation of T-cell activation via T cell receptor contact with antigen bound to MHC molecule on antigen presenting cell, regulation of T-lymphocyte activation via T cell receptor contact with antigen bound to MHC molecule on antigen presenting cell Definition: Any process that modulates the frequency, rate or extent of T cell activation via T cell receptor contact with antigen bound to MHC molecule on antigen presenting cell.